{
  "gene_symbol": "C20orf204",
  "term_label": "Unknown biological process",
  "gene": "UniProtKB:A0A1B0GTL2",
  "term_id": "UNKNOWN:0002",
  "gene_name": "Uncharacterized protein C20orf204"
}